{
  "gene": "UniProtKB:Q9UG63",
  "term_id": "GO:0005524",
  "gene_name": "ATP-binding cassette sub-family F member 2",
  "gene_symbol": "ABCF2",
  "term_label": "ATP binding"
}